pyruvate fermentation to acetate [GO:0019654] (biological process) Sources: GOC:jl, MetaCyc:P142-PWY Relationships: is a type of acetate metabolic process [GO:0006083]; is a type of pyruvate fermentation [GO:0019660] Also known as: acetate fermentation Definition: The anaerobic chemical reactions and pathways resulting in the breakdown of acetate, yielding energy in the form of ATP.